L-histidine catabolic process to glutamate and formamide [GO:0019556] (BP) Also known as: histidine catabolic process to glutamate and formamide, histidine breakdown to glutamate and formamide, histidine degradation to glutamate and formamide Definition: The chemical reactions and pathways resulting in the breakdown of L-histidine into other compounds, including glutamate and formamide. Sources: GOC:go_curators Relationships: is a type of GO:0006536; is a type of L-histidine catabolic process [GO:0006548]; is a type of amide catabolic process [GO:0043605]